{
  "term_label": "Golgi apparatus",
  "gene_name": "Coiled-coil domain-containing protein 170",
  "gene_symbol": "CCDC170",
  "gene": "UniProtKB:Q8IYT3",
  "term_id": "GO:0005794"
}